{
  "gene_symbol": "MED14",
  "term_id": "GO:0003712",
  "gene": "UniProtKB:O60244",
  "gene_name": "Mediator of RNA polymerase II transcription subunit 14",
  "term_label": "transcription coregulator activity"
}